{
  "gene_symbol": "SMARCA2",
  "gene_name": "Probable global transcription activator SNF2L2",
  "gene": "UniProtKB:P51531",
  "term_id": "GO:0045944",
  "term_label": "positive regulation of transcription by RNA polymerase II"
}